{
  "gene_symbol": "RNASE3",
  "gene_name": "Eosinophil cationic protein",
  "term_id": "UNKNOWN:0001",
  "gene": "UniProtKB:P12724",
  "term_label": "Unknown molecular function"
}